{
  "gene_symbol": "ZNF468",
  "term_label": "nucleus",
  "term_id": "GO:0005634",
  "gene": "UniProtKB:Q5VIY5",
  "gene_name": "Zinc finger protein 468"
}